{
  "term_label": "maturation of SSU-rRNA",
  "gene_name": "RNA-binding protein NOB1",
  "term_id": "GO:0030490",
  "gene_symbol": "NOB1",
  "gene": "UniProtKB:Q9ULX3"
}